{
  "gene_name": "G antigen 2B_2C",
  "gene": "UniProtKB:Q13066",
  "term_id": "UNKNOWN:0001",
  "gene_symbol": "GAGE2C",
  "term_label": "Unknown molecular function"
}